{
  "gene": "UniProtKB:P40425",
  "gene_symbol": "PBX2",
  "gene_name": "Pre-B-cell leukemia transcription factor 2",
  "term_label": "positive regulation of transcription by RNA polymerase II",
  "term_id": "GO:0045944"
}